{
  "term_label": "nucleus",
  "gene": "UniProtKB:O95801",
  "gene_symbol": "TTC4",
  "gene_name": "Tetratricopeptide repeat protein 4",
  "term_id": "GO:0005634"
}